{
  "term_label": "regulation of transcription by RNA polymerase II",
  "gene_symbol": "TBX2",
  "gene_name": "T-box transcription factor TBX2",
  "gene": "UniProtKB:Q13207",
  "term_id": "GO:0006357"
}